{
  "term_label": "signaling receptor binding",
  "term_id": "GO:0005102",
  "gene_symbol": "WIF1",
  "gene_name": "Wnt inhibitory factor 1",
  "gene": "UniProtKB:Q9Y5W5"
}